{
  "gene_symbol": "AGO2",
  "term_id": "GO:0005634",
  "term_label": "nucleus",
  "gene": "UniProtKB:Q9UKV8",
  "gene_name": "Protein argonaute-2"
}